{
  "gene_symbol": "ADH1C",
  "gene_name": "Alcohol dehydrogenase 1C",
  "term_id": "GO:0042572",
  "term_label": "retinol metabolic process",
  "gene": "UniProtKB:P00326"
}